positive regulation of cell junction assembly [GO:1901890] (biological process) Subtypes: positive regulation of focal adhesion assembly [GO:0051894], positive regulation of synapse assembly [GO:0051965], GO:1903348, GO:1903598 Relationships: is a type of positive regulation of cellular component biogenesis [GO:0044089]; is a type of positive regulation of cellular component organization [GO:0051130]; is a type of regulation of cell junction assembly [GO:1901888]; positively regulates cell junction assembly [GO:0034329] Also known as: up regulation of cell junction assembly, up-regulation of cell junction assembly, upregulation of cell junction assembly, activation of cell junction assembly Sources: GOC:TermGenie Definition: Any process that activates or increases the frequency, rate or extent of cell junction assembly.